TORC2 complex disassembly [GO:1905670] (biological process) References: PMID:21952218 Sources: GOC:TermGenie, GOC:kmv, GO_REF:0000079 Relationships: is a type of protein-containing complex disassembly [GO:0032984] Also known as: TOR complex 2 disassembly, TORC 2 complex disassembly, TORC2 disassembly, rapamycin and nutrient-insensitive TOR complex disassembly, mTORC2 disassembly Definition: The disaggregation of a TORC2 complex into its constituent components.